{
  "gene": "UniProtKB:Q86UK0",
  "term_label": "lipid transporter activity",
  "term_id": "GO:0005319",
  "gene_name": "Glucosylceramide transporter ABCA12",
  "gene_symbol": "ABCA12"
}